{
  "gene": "UniProtKB:P51164",
  "term_id": "GO:0030007",
  "gene_symbol": "ATP4B",
  "gene_name": "Potassium-transporting ATPase subunit beta",
  "term_label": "intracellular potassium ion homeostasis"
}